1-aminocyclopropane-1-carboxylate oxidase activity [GO:0009815] (molecular function) Definition: Catalysis of the reaction: 1-aminocyclopropane-1-carboxylate + L-ascorbate + O2 = CO2 + dehydroascorbate + ethylene + 2 H2O + hydrogen cyanide. Ethene is also known as ethylene. Sources: RHEA:23640 Also known as: ethene-forming enzyme, ethylene-forming enzyme, ACC oxidase activity, 1-aminocyclopropane-1-carboxylate oxygenase (ethylene-forming), aminocyclopropanecarboxylate oxidase activity Relationships: is a type of oxidoreductase activity, acting on paired donors, with incorporation or reduction of molecular oxygen, reduced ascorbate as one donor, and incorporation of one atom of oxygen [GO:0016715]